microtubule organizing center attachment site [GO:0034992] (cellular component) Definition: A region of the nuclear envelope to which a microtubule organizing center (MTOC) attaches; protein complexes embedded in the nuclear envelope mediate direct or indirect linkages between the microtubule cytoskeleton and the nuclear envelope. References: PMID:18692466 Sources: GOC:mah Also known as: MAS, MTOC attachment site, microtubule organising centre attachment site Note: Note that this term should not be confused with the cellular component term 'perinuclear region ; GO:0048471'. Relationships: is a type of GO:0110165; BFO_0000050 nuclear envelope [GO:0005635] Subtypes: GO:0180028